{
  "term_label": "Unknown cellular component",
  "term_id": "UNKNOWN:0003",
  "gene": "UniProtKB:Q15208",
  "gene_name": "Serine_threonine-protein kinase 38",
  "gene_symbol": "STK38"
}